{
  "term_id": "UNKNOWN:0001",
  "gene": "UniProtKB:B1ANY3",
  "term_label": "Unknown molecular function",
  "gene_name": "Putative protein FAM220BP",
  "gene_symbol": "FAM220BP"
}